peptidyl-glutamate ADP-deribosylation [GO:0140291] (biological process) Relationships: is a type of protein de-ADP-ribosylation [GO:0051725] Definition: The removal of ADP-ribose from ADP-ribosylglutamate. References: PMID:23481255